{
  "gene_name": "Nuclear factor NF-kappa-B p105 subunit",
  "gene": "UniProtKB:P19838",
  "gene_symbol": "NFKB1",
  "term_id": "GO:0000981",
  "term_label": "DNA-binding transcription factor activity, RNA polymerase II-specific"
}